compound eye corneal lens development [GO:0048058] (biological process) Sources: GOC:jid Relationships: is a type of anatomical structure development [GO:0048856]; is part of compound eye development [GO:0048749] Definition: The process whose specific outcome is the progression of the corneal lens in the compound eye over time, from its formation to the mature structure. The corneal lens is a chitinous extracellular secretion of the four underlying cone cells and the pigment cells.